{
  "gene_name": "Erythroid membrane-associated protein",
  "gene": "UniProtKB:Q96PL5",
  "gene_symbol": "ERMAP",
  "term_id": "GO:0005102",
  "term_label": "signaling receptor binding"
}